{
  "gene_symbol": "BPIFC",
  "term_id": "UNKNOWN:0002",
  "gene": "UniProtKB:Q8NFQ6",
  "term_label": "Unknown biological process",
  "gene_name": "BPI fold-containing family C protein"
}